{
  "gene": "UniProtKB:Q6PID8",
  "term_id": "GO:0032874",
  "gene_symbol": "KLHDC10",
  "gene_name": "Kelch domain-containing protein 10",
  "term_label": "positive regulation of stress-activated MAPK cascade"
}